positive regulation of stress-activated protein kinase signaling cascade [GO:0070304] (biological process) Subtypes: positive regulation of stress-activated MAPK cascade [GO:0032874] Also known as: positive regulation of SAPK signaling pathway, positive regulation of stress-activated protein kinase signaling pathway, positive regulation of stress-activated protein kinase signalling pathway, up regulation of stress-activated protein kinase signaling pathway, up-regulation of stress-activated protein kinase signaling pathway, upregulation of stress-activated protein kinase signaling pathway, activation of stress-activated protein kinase signaling pathway, stimulation of stress-activated protein kinase signaling pathway Definition: Any process that activates or increases the frequency, rate or extent of signaling via the stress-activated protein kinase signaling cascade. Relationships: is a type of regulation of stress-activated protein kinase signaling cascade [GO:0070302]; is a type of positive regulation of intracellular signal transduction [GO:1902533]; positively regulates GO:0031098 Sources: GOC:mah